tetrahydrofolate biosynthetic process [GO:0046654] (biological process) Relationships: is a type of GO:0009396; is a type of tetrahydrofolate metabolic process [GO:0046653] Subtypes: 10-formyltetrahydrofolate biosynthetic process [GO:0009257] Sources: ISBN:0198506732 Definition: The chemical reactions and pathways resulting in the formation of tetrahydrofolate, 5,6,7,8-tetrahydrofolic acid, a folate derivative bearing additional hydrogens on the pterin group. Also known as: tetrahydrofolate anabolism, tetrahydrofolate biosynthesis, tetrahydrofolate formation, tetrahydrofolate synthesis